{
  "gene_symbol": "RMND1",
  "gene_name": "Required for meiotic nuclear division protein 1 homolog",
  "term_id": "GO:0070131",
  "gene": "UniProtKB:Q9NWS8",
  "term_label": "positive regulation of mitochondrial translation"
}